{
  "term_label": "RNA helicase activity",
  "gene": "UniProtKB:Q9NXZ2",
  "term_id": "GO:0003724",
  "gene_name": "Probable ATP-dependent RNA helicase DDX43",
  "gene_symbol": "DDX43"
}